ribophagy [GO:0034517] (biological process) Definition: The selective degradation of mature ribosomes by macroautophagy. Relationships: is a type of GO:0016236 References: PMID:18391941 Sources: GOC:autophagy